{
  "gene_symbol": "SLC26A5",
  "gene_name": "Prestin",
  "gene": "UniProtKB:P58743",
  "term_id": "GO:0019531",
  "term_label": "oxalate transmembrane transporter activity"
}